{
  "term_id": "UNKNOWN:0002",
  "gene": "UniProtKB:O95153",
  "term_label": "Unknown biological process",
  "gene_symbol": "TSPOAP1",
  "gene_name": "Peripheral-type benzodiazepine receptor-associated protein 1"
}